{
  "gene": "UniProtKB:O14910",
  "term_id": "GO:0048489",
  "gene_symbol": "LIN7A",
  "gene_name": "Protein lin-7 homolog A",
  "term_label": "synaptic vesicle transport"
}